{
  "gene": "UniProtKB:Q8NB66",
  "term_id": "GO:0016081",
  "term_label": "synaptic vesicle docking",
  "gene_name": "Protein unc-13 homolog C",
  "gene_symbol": "UNC13C"
}